neuromedin B receptor binding [GO:0031710] (molecular function) Relationships: is a type of GO:0031705 Also known as: neuromedin B receptor ligand Sources: GOC:mah, GOC:nln Definition: Binding to a neuromedin B receptor.